{
  "gene_symbol": "HSPH1",
  "term_label": "protein folding",
  "gene_name": "Heat shock protein 105 kDa",
  "term_id": "GO:0006457",
  "gene": "UniProtKB:Q92598"
}